{
  "gene": "UniProtKB:Q96B97",
  "gene_symbol": "SH3KBP1",
  "term_label": "actin filament organization",
  "term_id": "GO:0007015",
  "gene_name": "SH3 domain-containing kinase-binding protein 1"
}